{
  "gene_symbol": "RETNLB",
  "term_id": "UNKNOWN:0002",
  "term_label": "Unknown biological process",
  "gene_name": "Resistin-like beta",
  "gene": "UniProtKB:Q9BQ08"
}